{
  "term_label": "alcohol dehydrogenase (NADP+) activity",
  "gene_name": "Aflatoxin B1 aldehyde reductase member 2",
  "gene_symbol": "AKR7A2",
  "term_id": "GO:0008106",
  "gene": "UniProtKB:O43488"
}